carboxyl- or carbamoyltransferase activity [GO:0016743] (molecular function) Sources: GOC:jl Also known as: carboxyl- and carbamoyltransferase activity Subtypes: aspartate carbamoyltransferase activity [GO:0004070], ornithine carbamoyltransferase activity [GO:0004585], GO:0043857, GO:0047154, 3-hydroxymethylcephem carbamoyltransferase activity [GO:0047155], lysine carbamoyltransferase activity [GO:0050068], oxamate carbamoyltransferase activity [GO:0050205], putrescine carbamoyltransferase activity [GO:0050231] Definition: Catalysis of the transfer of a carboxyl- or carbamoyl group from one compound (donor) to another (acceptor). Relationships: is a type of GO:0016741